{
  "term_label": "nuclear membrane reassembly",
  "gene_name": "Putative charged multivesicular body protein 4B-like protein CHMP4BP1",
  "gene_symbol": "CHMP4BP1",
  "gene": "UniProtKB:P59074",
  "term_id": "GO:0031468"
}